{
  "gene": "UniProtKB:Q8IVM8",
  "term_id": "UNKNOWN:0003",
  "gene_symbol": "SLC22A9",
  "gene_name": "Organic anion transporter 7",
  "term_label": "Unknown cellular component"
}